{
  "term_id": "GO:0048705",
  "gene_symbol": "RFLNB",
  "term_label": "skeletal system morphogenesis",
  "gene": "UniProtKB:Q8N5W9",
  "gene_name": "Refilin-B"
}